{
  "gene_symbol": "ZNF658B",
  "term_id": "GO:0000122",
  "gene_name": "Zinc finger protein 658B",
  "term_label": "negative regulation of transcription by RNA polymerase II",
  "gene": "UniProtKB:Q4V348"
}